{
  "gene_symbol": "PEAR1",
  "gene_name": "Platelet endothelial aggregation receptor 1",
  "term_label": "Unknown biological process",
  "term_id": "UNKNOWN:0002",
  "gene": "UniProtKB:Q5VY43"
}